{
  "gene": "UniProtKB:Q9Y5F7",
  "term_label": "synapse organization",
  "term_id": "GO:0050808",
  "gene_symbol": "PCDHGC4",
  "gene_name": "Protocadherin gamma-C4"
}